{
  "term_label": "nucleolus",
  "gene_name": "Transducin beta-like protein 3",
  "gene_symbol": "TBL3",
  "term_id": "GO:0005730",
  "gene": "UniProtKB:Q12788"
}